{
  "gene": "UniProtKB:Q9P2S6",
  "term_id": "UNKNOWN:0001",
  "term_label": "Unknown molecular function",
  "gene_name": "Ankyrin repeat and MYND domain-containing protein 1",
  "gene_symbol": "ANKMY1"
}